{
  "gene_name": "Copper transport protein ATOX1",
  "gene_symbol": "ATOX1",
  "term_id": "GO:0005829",
  "term_label": "cytosol",
  "gene": "UniProtKB:O00244"
}